{
  "gene_symbol": "ADAP1",
  "term_label": "Unknown biological process",
  "term_id": "UNKNOWN:0002",
  "gene_name": "Arf-GAP with dual PH domain-containing protein 1",
  "gene": "UniProtKB:O75689"
}